negative regulation of maintenance of mitotic sister chromatid cohesion [GO:0034183] (biological process) Subtypes: negative regulation of maintenance of mitotic sister chromatid cohesion, telomeric [GO:1904908], negative regulation of maintenance of mitotic sister chromatid cohesion, arms [GO:2000716], negative regulation of maintenance of mitotic sister chromatid cohesion, centromeric [GO:2000719] Definition: Any process that decreases the extent to which the association between sister chromatids of a replicated chromosome is maintained during a mitotic cell cycle. Sources: GOC:mah, GOC:vw Relationships: is a type of GO:0034092; is_a GO:0034182; RO_0002212 maintenance of mitotic sister chromatid cohesion [GO:0034088]